{
  "term_id": "GO:0008097",
  "gene_symbol": "NOP53",
  "gene": "UniProtKB:Q9NZM5",
  "gene_name": "Ribosome biogenesis protein NOP53",
  "term_label": "5S rRNA binding"
}